placental growth factor receptor activity [GO:0036332] (molecular function) References: PMID:12871269, PMID:7929268 Sources: GOC:uh, Wikipedia:Placental_growth_factor Definition: Combining with placental growth factor (PlGF) receptor ligand and transmitting the signal across the plasma membrane to initiate a change in cell activity. Relationships: is a type of GO:0004714; is part of GO:0036323 Also known as: PlGF-activated receptor activity, placental growth factor-activated receptor activity, PlGF receptor activity